{
  "term_label": "RNA polymerase II cis-regulatory region sequence-specific DNA binding",
  "gene_name": "T-box transcription factor TBX3",
  "term_id": "GO:0000978",
  "gene_symbol": "TBX3",
  "gene": "UniProtKB:O15119"
}